{
  "gene": "UniProtKB:A4FU01",
  "gene_name": "Myotubularin-related protein 11",
  "gene_symbol": "MTMR11",
  "term_label": "cytoplasm",
  "term_id": "GO:0005737"
}